{
  "gene_symbol": "ZNF355P",
  "gene_name": "Putative zinc finger protein 355P",
  "term_id": "GO:0005634",
  "gene": "UniProtKB:Q9NSJ1",
  "term_label": "nucleus"
}